ubiquitin-dependent endocytosis [GO:0070086] (biological process) Also known as: ubiquitin-mediated endocytosis Regulation: regulated by GO:2000395; negatively regulated by negative regulation of ubiquitin-dependent endocytosis [GO:2000396]; positively regulated by positive regulation of ubiquitin-dependent endocytosis [GO:2000397] Definition: Endocytosis of a protein that requires the substrate to be modified by ubiquitination. Several plasma membrane proteins, including cell surface permeases and some receptors, are targeted for internalization by endocytosis, and are thereafter delivered to the vacuole or lysosome, where they are degraded. Relationships: is a type of endocytosis [GO:0006897]; is_a protein transport [GO:0015031]; is a type of GO:0033365; is a type of GO:0072594 References: PMID:9409540 Sources: GOC:jp, GOC:mah